pregnan-21-ol dehydrogenase (NAD+) activity [GO:0047007] (molecular function) Relationships: is a type of steroid dehydrogenase activity, acting on the CH-OH group of donors, NAD or NADP as acceptor [GO:0033764] Definition: Catalysis of the reaction: NAD+ + pregnan-21-ol = H+ + NADH + pregnan-21-al. Sources: RHEA:11448 Also known as: 21-hydroxysteroid dehydrogenase (NAD+) activity, 21-hydroxysteroid:NAD+ 21-oxidoreductase activity